{
  "term_id": "GO:0005737",
  "term_label": "cytoplasm",
  "gene": "UniProtKB:Q6P1M3",
  "gene_symbol": "LLGL2",
  "gene_name": "LLGL scribble cell polarity complex component 2"
}